{
  "term_id": "GO:0035615",
  "term_label": "clathrin adaptor activity",
  "gene_symbol": "HIP1R",
  "gene": "UniProtKB:O75146",
  "gene_name": "Huntingtin-interacting protein 1-related protein"
}